{
  "gene_name": "Protein KIBRA",
  "term_label": "molecular adaptor activity",
  "gene": "UniProtKB:Q8IX03",
  "gene_symbol": "WWC1",
  "term_id": "GO:0060090"
}